{
  "gene_name": "Nuclear factor interleukin-3-regulated protein",
  "gene_symbol": "NFIL3",
  "term_id": "GO:0005634",
  "term_label": "nucleus",
  "gene": "UniProtKB:Q16649"
}